endosome membrane permeabilization involved in viral entry into host cell [GO:0075502] (BP) Sources: GOC:bf, GOC:jl Also known as: viral entry into host cell via caveolae-mediated endocytosis followed by endosome membrane, viral entry into host cell via clathrin-mediated endocytosis followed by endosome membrane permeabilization Definition: Induction of endosome membrane permeabilization triggered by an interaction between the host membrane and a membrane-penetration protein associated with the capsid. Occurs after internalization of the virus through the endosomal pathway, and results in delivery of the virus contents into the host cell cytoplasm. Relationships: is a type of permeabilization of host organelle membrane involved in viral entry into host cell [GO:0039665]